{
  "gene_symbol": "NXN",
  "term_id": "GO:0005634",
  "term_label": "nucleus",
  "gene": "UniProtKB:Q6DKJ4",
  "gene_name": "Nucleoredoxin"
}